{
  "gene_name": "Hyaluronan synthase 3",
  "gene_symbol": "HAS3",
  "term_label": "hyaluronan synthase activity",
  "gene": "UniProtKB:O00219",
  "term_id": "GO:0050501"
}